{
  "term_id": "GO:0051015",
  "gene_name": "Nebulette",
  "gene_symbol": "NEBL",
  "gene": "UniProtKB:O76041",
  "term_label": "actin filament binding"
}